negative regulation of intraciliary retrograde transport [GO:1905800] (biological process) References: PMID:27930654 Sources: GOC:TermGenie, GO_REF:0000058 Definition: Any process that stops, prevents or reduces the frequency, rate or extent of intraciliary retrograde transport. Also known as: down regulation of intraciliary retrograde transport, down regulation of intraflagellar retrograde transport, down-regulation of intraciliary retrograde transport, down-regulation of intraflagellar retrograde transport, downregulation of intraciliary retrograde transport, downregulation of intraflagellar retrograde transport, negative regulation of intraflagellar retrograde transport, inhibition of intraciliary retrograde transport, inhibition of intraflagellar retrograde transport Relationships: is a type of GO:0032387; is a type of regulation of intraciliary retrograde transport [GO:1905799]; negatively regulates intraciliary retrograde transport [GO:0035721]